{
  "gene": "UniProtKB:Q7L2Z9",
  "term_id": "GO:0051310",
  "gene_name": "Centromere protein Q",
  "gene_symbol": "CENPQ",
  "term_label": "metaphase chromosome alignment"
}